{
  "term_label": "protein de-ADP-ribosylation",
  "gene_symbol": "ADPRH",
  "gene": "UniProtKB:P54922",
  "gene_name": "ADP-ribosylhydrolase ARH1",
  "term_id": "GO:0051725"
}